cellular response to polycyclic arene [GO:1903166] (biological process) Subtypes: GO:1904682 Definition: Any process that results in a change in state or activity of a cell (in terms of movement, secretion, enzyme production, gene expression, etc.) as a result of a polycyclic arene stimulus. Relationships: is a type of cellular response to chemical stimulus [GO:0070887]; is a type of response to polycyclic arene [GO:1903165] References: PMID:10998501 Sources: GOC:TermGenie, GOC:mr, GO_REF:0000071